{
  "gene_name": "TBC domain-containing protein kinase-like protein",
  "gene_symbol": "TBCK",
  "term_label": "Unknown biological process",
  "term_id": "UNKNOWN:0002",
  "gene": "UniProtKB:Q8TEA7"
}